{
  "gene_symbol": "RAET1L",
  "gene_name": "UL16-binding protein 6",
  "term_label": "positive regulation of T cell mediated cytotoxicity",
  "gene": "UniProtKB:Q5VY80",
  "term_id": "GO:0001916"
}